{
  "term_label": "Unknown biological process",
  "gene_symbol": "OR4K14",
  "term_id": "UNKNOWN:0002",
  "gene": "UniProtKB:Q8NGD5",
  "gene_name": "Olfactory receptor 4K14"
}